{
  "term_label": "Unknown biological process",
  "gene_name": "Uncharacterized protein",
  "gene_symbol": "LOC102725191",
  "gene": "UniProtKB:A0A1B0GVB3",
  "term_id": "UNKNOWN:0002"
}